intracellular histidine homeostasis [GO:0090464] (biological process) Relationships: is a type of intracellular amino acid homeostasis [GO:0080144] Also known as: cellular histidine homeostasis, histidine homeostasis Sources: GOC:tb Definition: A homeostatic process involved in the maintenance of a steady state level of histidine within a cell.